{
  "gene": "UniProtKB:P0CJ74",
  "term_id": "GO:1900118",
  "term_label": "negative regulation of execution phase of apoptosis",
  "gene_symbol": "MTRNR2L7",
  "gene_name": "Humanin-like 7"
}